negative regulation of filamentous growth of a population of unicellular organisms in response to heat [GO:1900432] (biological process) Also known as: down regulation of filamentous growth of a population of unicellular organisms in response to heat, down-regulation of filamentous growth of a population of unicellular organisms in response to heat, downregulation of filamentous growth of a population of unicellular organisms in response to heat, inhibition of filamentous growth of a population of unicellular organisms in response to heat Sources: GOC:TermGenie, GOC:di Definition: Any process that stops, prevents or reduces the frequency, rate or extent of filamentous growth of a population of unicellular organisms in response to heat. Relationships: is a type of negative regulation of response to stimulus [GO:0048585]; is a type of negative regulation of filamentous growth of a population of unicellular organisms [GO:1900429]; is a type of regulation of filamentous growth of a population of unicellular organisms in response to heat [GO:1900431]; negatively regulates GO:0036168